{
  "term_id": "GO:0005801",
  "gene_symbol": "GOLGA8H",
  "term_label": "cis-Golgi network",
  "gene": "UniProtKB:P0CJ92",
  "gene_name": "Golgin subfamily A member 8H"
}